protein transport within plasma membrane [GO:0099632] (biological process) Sources: GOC:dos Relationships: is a type of protein transport within lipid bilayer [GO:0032594]; BFO_0000066 GO:0005886 Definition: A process in which protein is transported from one region of the plasma membrane to another. Subtypes: protein transport out of plasma membrane raft [GO:0044862]